toll-like receptor 12 signaling pathway [GO:0034174] (biological process) Also known as: TLR12 signaling pathway, toll-like receptor 12 signalling pathway References: PMID:16551253, PMID:17328678 Sources: GOC:add Relationships: is a type of GO:0140894 Definition: The series of molecular signals initiated by a ligand binding to the endolysosomal toll-like receptor 12. Regulation: RO_0002211 by GO:0034175; negatively regulated by GO:0034176; positively regulated by GO:0034177